{
  "term_label": "serine-type endopeptidase inhibitor activity",
  "gene": "UniProtKB:Q9H1F0",
  "term_id": "GO:0004867",
  "gene_symbol": "WFDC10A",
  "gene_name": "WAP four-disulfide core domain protein 10A"
}